SmD-containing SMN-Sm protein complex [GO:0034730] (cellular component) Relationships: is a type of SMN-Sm protein complex [GO:0034719] References: PMID:12975319, PMID:17401408 Definition: An SMN-Sm protein complex formed by the association of the methylated Sm proteins B/B', D1, D2, D3, E, F, and G with the SMN complex. Also known as: SMN-containing protein complex